{
  "term_id": "GO:0030154",
  "gene": "UniProtKB:Q3SYB3",
  "term_label": "cell differentiation",
  "gene_symbol": "FOXD4L6",
  "gene_name": "Forkhead box protein D4-like 6"
}